pyruvate oxidase (CoA-acetylating) activity [GO:0050244] (molecular function) Sources: RHEA:21912 Definition: Catalysis of the reaction: CoA + H+ + O2 + pyruvate = acetyl-CoA + CO2 + H2O2. Relationships: is a type of GO:0016623 Also known as: pyruvate:oxygen 2-oxidoreductase (CoA-acetylating)